phosphatidylserine catabolic process [GO:0006660] (biological process) Definition: The chemical reactions and pathways resulting in the breakdown of phosphatidylserines, any of a class of glycerophospholipids in which the phosphatidyl group is esterified to the hydroxyl group of L-serine. Also known as: phosphatidylserine breakdown, phosphatidylserine catabolism, phosphatidylserine degradation Relationships: is a type of phosphatidylserine metabolic process [GO:0006658]; is a type of GO:0042219; is a type of glycerophospholipid catabolic process [GO:0046475] Sources: ISBN:0198506732